{
  "term_label": "phosphatidylinositol transfer activity",
  "gene": "UniProtKB:Q5GJ75",
  "gene_symbol": "TNFAIP8L3",
  "term_id": "GO:0008526",
  "gene_name": "Tumor necrosis factor alpha-induced protein 8-like protein 3"
}